regulation of transdifferentiation [GO:1903618] (biological process) References: PMID:22118091 Sources: GOC:TermGenie, GO_REF:0000058 Definition: Any process that modulates the frequency, rate or extent of transdifferentiation. Subtypes: negative regulation of transdifferentiation [GO:1903619], positive regulation of transdifferentiation [GO:1903620] Relationships: is a type of GO:0045595; regulates transdifferentiation [GO:0060290]